{
  "gene_name": "Homeobox protein Hox-C11",
  "gene_symbol": "HOXC11",
  "term_label": "regulation of transcription by RNA polymerase II",
  "gene": "UniProtKB:O43248",
  "term_id": "GO:0006357"
}